{
  "gene_symbol": "SGO1",
  "gene": "UniProtKB:Q5FBB7",
  "gene_name": "Shugoshin 1",
  "term_label": "meiotic sister chromatid cohesion",
  "term_id": "GO:0051177"
}